{
  "term_label": "potassium:proton antiporter activity",
  "term_id": "GO:0015386",
  "gene_symbol": "SLC9A8",
  "gene": "UniProtKB:Q9Y2E8",
  "gene_name": "Sodium_hydrogen exchanger 8"
}